{
  "term_label": "endoplasmic reticulum membrane",
  "gene": "UniProtKB:Q12907",
  "term_id": "GO:0005789",
  "gene_symbol": "LMAN2",
  "gene_name": "Vesicular integral-membrane protein VIP36"
}